{
  "term_label": "DNA-binding transcription factor activity, RNA polymerase II-specific",
  "gene": "UniProtKB:Q68EA5",
  "gene_symbol": "ZNF57",
  "term_id": "GO:0000981",
  "gene_name": "Zinc finger protein 57"
}